{
  "gene_name": "Putative DBH-like monooxygenase protein 2",
  "gene": "UniProtKB:A6NHM9",
  "term_label": "dopamine beta-monooxygenase activity",
  "gene_symbol": "MOXD2P",
  "term_id": "GO:0004500"
}